regulation of trans-synaptic signaling [GO:0099177] (BP) Sources: GOC:dos Definition: Any process that modulates the frequency, rate or extent of trans-synaptic signaling. Subtypes: GO:0050804, regulation of retrograde trans-synaptic signaling by trans-synaptic protein complex [GO:0099176], regulation of retrograde trans-synaptic signaling by endocanabinoid [GO:0099178], regulation of retrograde trans-synaptic signaling by neuropeptide [GO:1905432] Relationships: is a type of GO:0010646; is a type of regulation of signaling [GO:0023051]; regulates trans-synaptic signaling [GO:0099537]